{
  "gene_name": "Secreted frizzled-related protein 4",
  "term_id": "GO:0035567",
  "gene_symbol": "SFRP4",
  "gene": "UniProtKB:Q6FHJ7",
  "term_label": "non-canonical Wnt signaling pathway"
}